{
  "term_label": "Unknown cellular component",
  "gene_name": "Uncharacterized protein C22orf15",
  "gene": "UniProtKB:Q8WYQ4",
  "gene_symbol": "C22orf15",
  "term_id": "UNKNOWN:0003"
}